{
  "gene_symbol": "CRLS1",
  "gene": "UniProtKB:Q9UJA2",
  "term_label": "mitochondrion",
  "term_id": "GO:0005739",
  "gene_name": "Cardiolipin synthase (CMP-forming)"
}